{
  "gene_symbol": "HAS1",
  "term_label": "extracellular matrix assembly",
  "gene": "UniProtKB:Q92839",
  "term_id": "GO:0085029",
  "gene_name": "Hyaluronan synthase 1"
}